sporulation [GO:0043934] (biological process) Sources: GOC:pamgo_curators Subtypes: sporulation resulting in formation of a cellular spore [GO:0030435], GO:0030436, sexual sporulation [GO:0034293], sporulation resulting in formation of a multicellular or syncytial spore [GO:0075283] Definition: The process whose specific outcome is the progression of a spore over time, from its initiation to the mature structure. A spore is a structure that can be used for dissemination, for survival of adverse conditions because of its heat and desiccation resistance, and/or for reproduction. Relationships: is a type of GO:0032502 Regulation: regulated by regulation of sporulation [GO:0043937]; positively regulated by positive regulation of sporulation [GO:0043938]; negatively regulated by GO:0043939